{
  "gene": "UniProtKB:Q99424",
  "term_id": "GO:0000038",
  "gene_symbol": "ACOX2",
  "term_label": "very long-chain fatty acid metabolic process",
  "gene_name": "Peroxisomal acyl-coenzyme A oxidase 2"
}